{
  "term_label": "autophagosome",
  "gene_symbol": "TP53INP2",
  "gene_name": "Tumor protein p53-inducible nuclear protein 2",
  "gene": "UniProtKB:Q8IXH6",
  "term_id": "GO:0005776"
}